{
  "term_id": "UNKNOWN:0003",
  "gene": "UniProtKB:Q14BN4",
  "gene_symbol": "SLMAP",
  "gene_name": "Sarcolemmal membrane-associated protein",
  "term_label": "Unknown cellular component"
}